{
  "gene": "UniProtKB:Q8N5H7",
  "gene_symbol": "SH2D3C",
  "gene_name": "SH2 domain-containing protein 3C",
  "term_id": "UNKNOWN:0003",
  "term_label": "Unknown cellular component"
}